{
  "gene_name": "Clathrin interactor 1",
  "term_label": "plasma membrane",
  "gene": "UniProtKB:Q14677",
  "gene_symbol": "CLINT1",
  "term_id": "GO:0005886"
}